{
  "term_label": "signal peptide processing",
  "gene_symbol": "FURIN",
  "term_id": "GO:0006465",
  "gene_name": "Furin",
  "gene": "UniProtKB:P09958"
}